histone phosphatase activity [GO:0140789] (molecular function) Relationships: is a type of phosphoprotein phosphatase activity [GO:0004721]; is a type of histone modifying activity [GO:0140993] Subtypes: histone H2AXS139 phosphatase activity [GO:0140791], histone H2AXY142 phosphatase activity [GO:0140793] References: PMID:19351884 Definition: Catalysis of the reaction: a phosphorylated histone + H2O = a protein + phosphate.